{
  "term_label": "mitochondrion",
  "term_id": "GO:0005739",
  "gene_name": "Uncharacterized aarF domain-containing protein kinase 2",
  "gene_symbol": "ADCK2",
  "gene": "UniProtKB:Q7Z695"
}